{
  "gene_symbol": "CLUHP3",
  "gene": "UniProtKB:Q96NS8",
  "term_label": "Unknown biological process",
  "term_id": "UNKNOWN:0002",
  "gene_name": "Putative protein CLUHP3"
}